{
  "gene_symbol": "TIMP2",
  "gene": "UniProtKB:P16035",
  "gene_name": "Metalloproteinase inhibitor 2",
  "term_label": "response to hormone",
  "term_id": "GO:0009725"
}